propionyl-CoA metabolic process [GO:1902858] (biological process) Also known as: propionyl-CoA metabolism Relationships: is a type of GO:0035337 References: PMID:15514053 Sources: GOC:TermGenie, GOC:mengo_curators, GO_REF:0000068 Subtypes: propionyl-CoA catabolic process [GO:1902859], propionyl-CoA biosynthetic process [GO:1902860] Definition: The chemical reactions and pathways involving propionyl-CoA.